{
  "gene_name": "Sorting nexin-17",
  "term_id": "GO:0035091",
  "gene_symbol": "SNX17",
  "gene": "UniProtKB:Q15036",
  "term_label": "phosphatidylinositol binding"
}